{
  "gene": "UniProtKB:P17509",
  "term_id": "GO:0006357",
  "term_label": "regulation of transcription by RNA polymerase II",
  "gene_symbol": "HOXB6",
  "gene_name": "Homeobox protein Hox-B6"
}